{
  "term_label": "guanyl-nucleotide exchange factor activity",
  "term_id": "GO:0005085",
  "gene": "UniProtKB:A0A590UK10",
  "gene_symbol": "ARHGEF18",
  "gene_name": "Rho guanine nucleotide exchange factor 18 (Fragment)"
}